{
  "term_label": "negative regulation of apoptotic process",
  "gene_name": "Wilms tumor protein",
  "term_id": "GO:0043066",
  "gene_symbol": "WT1",
  "gene": "UniProtKB:P19544"
}